{
  "term_id": "GO:0005634",
  "gene_name": "Cyclin-dependent kinase 20",
  "gene": "UniProtKB:Q8IZL9",
  "term_label": "nucleus",
  "gene_symbol": "CDK20"
}